cytidine metabolic process [GO:0046087] (biological process) Definition: The chemical reactions and pathways involving cytidine, cytosine riboside, a widely distributed nucleoside. Sources: GOC:go_curators Also known as: cytidine metabolism Relationships: is a type of pyrimidine ribonucleoside metabolic process [GO:0046131] Subtypes: cytidine catabolic process [GO:0006216]